symbiont-mediated perturbation of host receptor-mediated endocytosis [GO:0044077] (biological process) Definition: A process in which a symbiont initiates, promotes, or enhances host receptor-mediated endocytosis, the uptake of external materials by cells, utilizing receptors to ensure specificity of transport. The host is defined as the larger of the organisms involved in a symbiotic interaction. Also known as: modulation by symbiont of host receptor-mediated endocytosis, modulation of host receptor-mediated endocytosis by symbiont, regulation by symbiont of host receptor-mediated endocytosis Relationships: is a type of symbiont-mediated perturbation of host vesicle-mediated transport [GO:1990215] Sources: MITRE:tk